{
  "term_label": "cellular response to starvation",
  "gene": "UniProtKB:Q7L523",
  "term_id": "GO:0009267",
  "gene_name": "Ras-related GTP-binding protein A",
  "gene_symbol": "RRAGA"
}